cell-cell adhesion involved in cerebral cortex tangential migration using cell-cell interactions [GO:0021832] (biological process) Relationships: is a type of GO:0098609; is part of cerebral cortex tangential migration using cell-cell interactions [GO:0021823] References: PMID:12626695 Sources: GOC:cls, GOC:dgh, GOC:dph, GOC:jid, GO_REF:0000021 Definition: The attachment of cells to one another to form groups of cells involved in cerebral cortex tangential migration.